{
  "term_label": "Golgi apparatus",
  "gene_name": "Probable palmitoyltransferase ZDHHC24",
  "term_id": "GO:0005794",
  "gene": "UniProtKB:Q6UX98",
  "gene_symbol": "ZDHHC24"
}